{
  "gene_name": "Frizzled-1",
  "gene_symbol": "FZD1",
  "term_label": "plasma membrane",
  "term_id": "GO:0005886",
  "gene": "UniProtKB:Q9UP38"
}